{
  "term_label": "negative regulation of smoothened signaling pathway",
  "gene": "UniProtKB:Q9Y6C5",
  "gene_symbol": "PTCH2",
  "gene_name": "Protein patched homolog 2",
  "term_id": "GO:0045879"
}